{
  "term_label": "cytoplasm",
  "gene_name": "Lamin tail domain-containing protein 1",
  "term_id": "GO:0005737",
  "gene_symbol": "LMNTD1",
  "gene": "UniProtKB:Q8N9Z9"
}